{
  "gene_name": "Syntaxin-binding protein 3",
  "gene_symbol": "STXBP3",
  "term_id": "GO:0005886",
  "term_label": "plasma membrane",
  "gene": "UniProtKB:O00186"
}